fatty-acyl-ethyl-ester synthase activity [GO:0030339] (MF) Definition: Catalysis of the reaction: a long-chain-acyl ethyl ester + H2O = a long-chain carboxylic acid + ethanol. Also known as: fatty-acyl ethyl ester synthase, FAEE synthase activity, FAEES activity, long-chain-fatty-acyl-ethyl-ester acylhydrolase activity Relationships: is a type of GO:0052689 Sources: EC:3.1.1.67